{
  "gene_symbol": "BHLHE40",
  "term_label": "circadian regulation of gene expression",
  "gene_name": "Class E basic helix-loop-helix protein 40",
  "gene": "UniProtKB:O14503",
  "term_id": "GO:0032922"
}